{
  "gene": "UniProtKB:Q5H9E4",
  "term_id": "GO:0051724",
  "gene_name": "Solute carrier family 25 member 53",
  "gene_symbol": "SLC25A53",
  "term_label": "NAD transmembrane transporter activity"
}